{
  "term_id": "UNKNOWN:0002",
  "gene_name": "Protein MANBAL",
  "gene_symbol": "MANBAL",
  "gene": "UniProtKB:Q9NQG1",
  "term_label": "Unknown biological process"
}